regulation of developmental process [GO:0050793] (biological process) Definition: Any process that modulates the frequency, rate or extent of development, the biological process whose specific outcome is the progression of a multicellular organism over time from an initial condition (e.g. a zygote, or a young adult) to a later condition (e.g. a multicellular animal or an aged adult). Relationships: is a type of regulation of biological process [GO:0050789]; regulates developmental process [GO:0032502] Subtypes: regulation of meristem structural organization [GO:0009934], regulation of cell fate commitment [GO:0010453], GO:0022603, GO:0031156, regulation of mating projection assembly [GO:0031383], GO:0031494, regulation of hemocyte proliferation [GO:0035206], regulation of vulval development [GO:0040028], regulation of development, heterochronic [GO:0040034], regulation of sporulation [GO:0043937], regulation of cell differentiation [GO:0045595], GO:0045682, regulation of salivary gland boundary specification [GO:0045704], regulation of retinal cell programmed cell death [GO:0046668], GO:0048088, regulation of female pigmentation [GO:0048089], regulation of meristem development [GO:0048509], regulation of muscle organ development [GO:0048634], regulation of developmental growth [GO:0048638], regulation of hair follicle maturation [GO:0048819], regulation of shoot system development [GO:0048831], specification of plant organ number [GO:0048832], regulation of dendrite development [GO:0050773], negative regulation of developmental process [GO:0051093], positive regulation of developmental process [GO:0051094], regulation of syncytium formation by plasma membrane fusion [GO:0060142], regulation of aggregation involved in sorocarp development [GO:0060176], regulation of floral organ abscission [GO:0060860], regulation of dendritic spine development [GO:0060998], regulation of neural retina development [GO:0061074], regulation of dermatome development [GO:0061183], GO:0061190, regulation of entry into reproductive diapause [GO:0061963], regulation of somatic muscle development [GO:0062223], regulation of neuron projection regeneration [GO:0070570], regulation of conidiophore stalk development [GO:0070799], regulation of germ tube formation [GO:0075010], modulation of formation of symbiont germ tube hook structure for appressorium development [GO:0075030], modulation of penetration peg formation [GO:0075054], regulation of infection cushion formation [GO:0075184], regulation of haustorium mother cell formation [GO:0075193], GO:0075198, regulation of spore-bearing organ development [GO:0075260], regulation of synapse maturation [GO:0090128], GO:0090183, regulation of blastocyst development [GO:0120222], GO:1900055, regulation of bone trabecula formation [GO:1900154], regulation of pronephric nephron tubule development [GO:1900206], regulation of cardiac chamber formation [GO:1901210], GO:1901861, GO:1901922, regulation of embryonic skeletal joint development [GO:1902762], GO:1902863, GO:1902866, regulation of ascospore-type prospore membrane formation [GO:1903023], regulation of tube lumen cavitation [GO:1903132], regulation of adipose tissue development [GO:1904177], GO:1904248, regulation of spore germination [GO:1904359], regulation of cardiac ventricle development [GO:1904412], GO:1904653, regulation of apoptotic process involved in development [GO:1904748], GO:1905174, regulation of mesoderm formation [GO:1905902], regulation of cell fate determination [GO:1905933], GO:1905939, regulation of endosperm development [GO:2000014], GO:2000024, GO:2000026, regulation of stem cell population maintenance [GO:2000036], regulation of root development [GO:2000280], regulation of myotome development [GO:2000290], regulation of blood microparticle formation [GO:2000332], regulation of ovarian follicle development [GO:2000354], regulation of mesoderm development [GO:2000380], regulation of ectoderm development [GO:2000383], regulation of anterior head development [GO:2000742] Sources: GOC:go_curators